endocytic patch [GO:0061645] (CC) Subtypes: actin cortical patch [GO:0030479] Relationships: is a type of cellular anatomical structure [GO:0110165]; is part of cell cortex [GO:0005938] References: PMID:22949647 Sources: GOC:dph Definition: The part of the cell cortex consisting of an aggregation of proteins that will give rise to an endocytic vesicle.